intracellular mRNA localization involved in pattern specification process [GO:0060810] (biological process) Sources: GOC:dph, GOC:sdb_2009, GOC:tb Definition: Any process in which mRNA is transported to, or maintained in, a specific location within an oocyte that results in a pattern being established in the embryo. Also known as: intracellular mRNA localisation involved in pattern specification process Relationships: is a type of intracellular mRNA localization [GO:0008298]; is part of pattern specification process [GO:0007389] Subtypes: intracellular mRNA localization involved in anterior/posterior axis specification [GO:0060811]